{
  "gene_symbol": "KIF16B",
  "term_label": "cytoplasm",
  "term_id": "GO:0005737",
  "gene_name": "Kinesin-like protein KIF16B",
  "gene": "UniProtKB:Q96L93"
}